positive regulation of dipeptide transmembrane transport [GO:2001150] (biological process) Definition: Any process that activates or increases the frequency, rate or extent of dipeptide transmembrane transport. Relationships: is a type of positive regulation of transmembrane transport [GO:0034764]; is a type of positive regulation of dipeptide transport [GO:2000880]; is a type of regulation of dipeptide transmembrane transport [GO:2001148]; positively regulates dipeptide transmembrane transport [GO:0035442] Also known as: positive regulation of dipeptide membrane transport Sources: GOC:obol